post-embryonic hindgut morphogenesis [GO:0048620] (biological process) Sources: GOC:jid, GOC:rc Relationships: is a type of post-embryonic animal morphogenesis [GO:0009886]; is part of hindgut morphogenesis [GO:0007442] Definition: The process in which the anatomical structures of the hindgut are generated and organized, during the post-embryonic phase.